{
  "gene_symbol": "VMP1",
  "gene_name": "Vacuole membrane protein 1",
  "term_label": "endoplasmic reticulum",
  "gene": "UniProtKB:Q96GC9",
  "term_id": "GO:0005783"
}